positive regulation of epithelial cell apoptotic process [GO:1904037] (biological process) References: PMID:19137015 Sources: GOC:TermGenie, GO_REF:0000058 Definition: Any process that activates or increases the frequency, rate or extent of epithelial cell apoptotic process. Relationships: is a type of positive regulation of apoptotic process [GO:0043065]; is_a GO:1904035; positively regulates epithelial cell apoptotic process [GO:1904019] Subtypes: positive regulation of keratinocyte apoptotic process [GO:1902174], positive regulation of hepatocyte apoptotic process [GO:1903945], positive regulation of cholangiocyte apoptotic process [GO:1904194], positive regulation of podocyte apoptotic process [GO:1904635], positive regulation of granulosa cell apoptotic process [GO:1904710], GO:2000676 Also known as: positive regulation of epitheliocyte apoptotic process, up regulation of epithelial cell apoptotic process, up regulation of epitheliocyte apoptotic process, up-regulation of epithelial cell apoptotic process, up-regulation of epitheliocyte apoptotic process, upregulation of epithelial cell apoptotic process, upregulation of epitheliocyte apoptotic process, activation of epithelial cell apoptosis, activation of epithelial cell apoptotic process, activation of epitheliocyte apoptosis, activation of epitheliocyte apoptotic process, positive regulation of epithelial cell apoptosis, positive regulation of epitheliocyte apoptosis, up regulation of epithelial cell apoptosis, up regulation of epitheliocyte apoptosis, up-regulation of epithelial cell apoptosis, up-regulation of epitheliocyte apoptosis, upregulation of epithelial cell apoptosis, upregulation of epitheliocyte apoptosis